{
  "term_id": "GO:0005886",
  "gene_symbol": "FZD7",
  "gene_name": "Frizzled-7",
  "gene": "UniProtKB:O75084",
  "term_label": "plasma membrane"
}